{
  "term_label": "endosome",
  "term_id": "GO:0005768",
  "gene": "UniProtKB:Q86XR7",
  "gene_symbol": "TICAM2",
  "gene_name": "TIR domain-containing adapter molecule 2"
}